{
  "gene_symbol": "IL9",
  "gene_name": "Interleukin-9",
  "term_label": "extracellular space",
  "gene": "UniProtKB:P15248",
  "term_id": "GO:0005615"
}